{
  "gene_name": "Protein salvador homolog 1",
  "gene_symbol": "SAV1",
  "gene": "UniProtKB:Q9H4B6",
  "term_id": "GO:0043065",
  "term_label": "positive regulation of apoptotic process"
}